{
  "term_label": "glycolytic process",
  "term_id": "GO:0006096",
  "gene": "UniProtKB:P19367",
  "gene_name": "Hexokinase-1",
  "gene_symbol": "HK1"
}